{
  "term_id": "GO:0090385",
  "gene_symbol": "RAB7B",
  "term_label": "phagosome-lysosome fusion",
  "gene_name": "Ras-related protein Rab-7b",
  "gene": "UniProtKB:Q96AH8"
}